{
  "term_id": "GO:0051321",
  "gene_name": "Replication protein A 70 kDa DNA-binding subunit",
  "gene": "UniProtKB:P27694",
  "term_label": "meiotic cell cycle",
  "gene_symbol": "RPA1"
}